{
  "gene_name": "Leucine-rich repeats and immunoglobulin-like domains protein 1",
  "term_label": "signaling receptor activity",
  "gene_symbol": "LRIG1",
  "gene": "UniProtKB:Q96JA1",
  "term_id": "GO:0038023"
}